pyrimidine ribonucleoside diphosphate biosynthetic process [GO:0009194] (biological process) Definition: The chemical reactions and pathways resulting in the formation of pyrimidine ribonucleoside diphosphate, a compound consisting of a pyrimidine base linked to a ribose sugar esterified with diphosphate on the sugar. Relationships: is a type of GO:0009139; is a type of ribonucleoside diphosphate biosynthetic process [GO:0009188]; is a type of GO:0009193 Also known as: pyrimidine ribonucleoside diphosphate anabolism, pyrimidine ribonucleoside diphosphate biosynthesis, pyrimidine ribonucleoside diphosphate formation, pyrimidine ribonucleoside diphosphate synthesis Subtypes: GO:0006225, TDP biosynthetic process [GO:0006232], CDP biosynthetic process [GO:0046705] Sources: GOC:go_curators, ISBN:0198506732